plant epidermal cell differentiation [GO:0090627] (biological process) Relationships: is a type of GO:0030154 Regulation: regulated by regulation of plant epidermal cell differentiation [GO:1903888]; RO_0002212 by negative regulation of plant epidermal cell differentiation [GO:1903889]; positively regulated by positive regulation of plant epidermal cell differentiation [GO:1903890] Sources: GOC:tb Subtypes: guard cell differentiation [GO:0010052], root epidermal cell differentiation [GO:0010053], guard mother cell differentiation [GO:0010444], sepal giant cell differentiation [GO:0090392], GO:0090437 Definition: The process in which a relatively unspecialized cell acquires specialized features of a plant epidermal cell.